{
  "term_label": "angiotensin maturation",
  "gene": "UniProtKB:Q9BYF1",
  "gene_symbol": "ACE2",
  "gene_name": "Angiotensin-converting enzyme 2",
  "term_id": "GO:0002003"
}